{
  "gene": "UniProtKB:Q9NPD5",
  "gene_name": "Solute carrier organic anion transporter family member 1B3",
  "term_label": "bile acid and bile salt transport",
  "gene_symbol": "SLCO1B3",
  "term_id": "GO:0015721"
}